{
  "gene": "UniProtKB:O94927",
  "gene_name": "HAUS augmin-like complex subunit 5",
  "gene_symbol": "HAUS5",
  "term_id": "GO:0051225",
  "term_label": "spindle assembly"
}